{
  "term_label": "synapse",
  "gene_symbol": "CYFIP1",
  "gene_name": "Cytoplasmic FMR1-interacting protein 1",
  "gene": "UniProtKB:Q7L576",
  "term_id": "GO:0045202"
}